{
  "gene_name": "G-protein coupled receptor family C group 5 member B",
  "gene_symbol": "GPRC5B",
  "gene": "UniProtKB:Q9NZH0",
  "term_label": "Unknown biological process",
  "term_id": "UNKNOWN:0002"
}